{
  "gene_name": "Anaphase-promoting complex subunit 10",
  "gene_symbol": "ANAPC10",
  "gene": "UniProtKB:Q9UM13",
  "term_label": "Unknown molecular function",
  "term_id": "UNKNOWN:0001"
}